{
  "gene_name": "Protein mono-ADP-ribosyltransferase PARP8",
  "gene": "UniProtKB:Q8N3A8",
  "gene_symbol": "PARP8",
  "term_id": "GO:0005635",
  "term_label": "nuclear envelope"
}